{
  "gene_symbol": "ARPC3",
  "gene_name": "Actin-related protein 2_3 complex subunit 3",
  "gene": "UniProtKB:O15145",
  "term_label": "Arp2/3 protein complex",
  "term_id": "GO:0005885"
}